pyridoxine import across plasma membrane [GO:1903075] (biological process) References: PMID:15701794 Sources: GOC:TermGenie, GO_REF:0000075 Also known as: pyridoxine import into cell Relationships: is a type of import across plasma membrane [GO:0098739]; is_a pyridoxine transmembrane transport [GO:1903092] Definition: The directed movement of pyridoxine from outside of a cell, across the plasma membrane and into the cytosol.